neutrophil chemotaxis [GO:0030593] (biological process) Sources: GOC:jl, ISBN:0198506732 Regulation: regulated by GO:0090022; positively regulated by positive regulation of neutrophil chemotaxis [GO:0090023]; negatively regulated by GO:0090024 Definition: The directed movement of a neutrophil cell, the most numerous polymorphonuclear leukocyte found in the blood, in response to an external stimulus, usually an infection or wounding. Relationships: is a type of granulocyte chemotaxis [GO:0071621]; is a type of neutrophil migration [GO:1990266]